{
  "term_label": "extracellular space",
  "gene_name": "SPARC-like protein 1",
  "term_id": "GO:0005615",
  "gene": "UniProtKB:Q14515",
  "gene_symbol": "SPARCL1"
}